{
  "gene_name": "Cyclic AMP-dependent transcription factor ATF-1",
  "gene": "UniProtKB:P18846",
  "term_id": "GO:1990589",
  "gene_symbol": "ATF1",
  "term_label": "ATF4-CREB1 transcription factor complex"
}